{
  "gene": "UniProtKB:O15350",
  "term_id": "GO:0045944",
  "term_label": "positive regulation of transcription by RNA polymerase II",
  "gene_name": "Tumor protein p73",
  "gene_symbol": "TP73"
}